{
  "gene": "UniProtKB:P0CG42",
  "gene_name": "Putative protein FAM157B",
  "term_id": "UNKNOWN:0001",
  "gene_symbol": "FAM157B",
  "term_label": "Unknown molecular function"
}